8-oxo-dGDP phosphatase activity [GO:0044715] (molecular function) Relationships: is a type of GO:0017110 References: PMID:22556419 Sources: GOC:pde, RHEA:32063 Definition: Catalysis of the reaction 8-oxo-dGDP + H2O = 8-oxo-dGMP + phosphate.